{
  "term_label": "Unknown cellular component",
  "gene_symbol": "HS3ST4",
  "gene_name": "Heparan sulfate glucosamine 3-O-sulfotransferase 4",
  "gene": "UniProtKB:Q9Y661",
  "term_id": "UNKNOWN:0003"
}